{
  "term_id": "UNKNOWN:0001",
  "gene": "UniProtKB:Q6UWW9",
  "term_label": "Unknown molecular function",
  "gene_name": "Transmembrane protein 207",
  "gene_symbol": "TMEM207"
}